{
  "gene_name": "Homeobox-containing protein 1",
  "term_id": "UNKNOWN:0002",
  "gene_symbol": "HMBOX1",
  "gene": "UniProtKB:Q6NT76",
  "term_label": "Unknown biological process"
}